{
  "gene": "UniProtKB:Q96SN8",
  "gene_name": "CDK5 regulatory subunit-associated protein 2",
  "term_label": "establishment of mitotic spindle orientation",
  "gene_symbol": "CDK5RAP2",
  "term_id": "GO:0000132"
}